{
  "term_id": "UNKNOWN:0001",
  "gene": "UniProtKB:Q13740",
  "gene_name": "CD166 antigen",
  "gene_symbol": "ALCAM",
  "term_label": "Unknown molecular function"
}